phenylethylamine metabolic process [GO:0042443] (biological process) Definition: The chemical reactions and pathways involving phenylethylamine, an amine with pharmacological properties similar to those of amphetamine, occurs naturally as a neurotransmitter in the brain, and is present in chocolate and oil of bitter almonds. Sources: GOC:jl, ISBN:0395825172 Subtypes: phenylethylamine catabolic process [GO:0019607], phenylethylamine biosynthetic process [GO:0042444] Relationships: is a type of biogenic amine metabolic process [GO:0006576] Also known as: phenylethylamine metabolism